chitobiose catabolic process [GO:0052781] (biological process) Definition: The chemical reactions and pathways resulting in the breakdown of any chitobiose, a family of compounds derived from chitin and based on the structure of D-glucosaminyl-(1->4)-D-glucosamine. Relationships: is a type of catabolic process [GO:0009056]; is a type of carbohydrate derivative metabolic process [GO:1901135] Sources: GOC:curators